{
  "gene_name": "GATOR complex protein NPRL2",
  "gene": "UniProtKB:Q8WTW4",
  "gene_symbol": "NPRL2",
  "term_id": "UNKNOWN:0001",
  "term_label": "Unknown molecular function"
}